mRNA export from nucleus in response to heat stress [GO:0031990] (BP) Relationships: is a type of mRNA export from nucleus [GO:0006406]; is a type of cellular response to heat [GO:0034605]; is a type of GO:1901698 Regulation: regulated by regulation of mRNA export from nucleus in response to heat stress [GO:2000728] Definition: The directed movement of mRNA from the nucleus to the cytoplasm during a heat stimulus, a temperature stimulus above the optimal temperature for the organism; in particular, a process that enables an organism withstand exposure to temperatures that would otherwise lethally impair poly(A)+ mRNA-nucleus export. Sources: GOC:mah, GOC:vw Also known as: mRNA export from cell nucleus during heat stress, mRNA export from nucleus during heat stress